{
  "gene_symbol": "JARID2",
  "gene_name": "Protein Jumonji",
  "gene": "UniProtKB:Q92833",
  "term_id": "GO:0010468",
  "term_label": "regulation of gene expression"
}